{
  "gene_symbol": "TEK",
  "term_id": "GO:0045766",
  "gene_name": "Angiopoietin-1 receptor",
  "term_label": "positive regulation of angiogenesis",
  "gene": "UniProtKB:Q02763"
}